olfactory learning [GO:0008355] (BP) Regulation: regulated by regulation of olfactory learning [GO:0090328] Sources: ISBN:0582227089 Definition: Any process in an organism in which a relatively long-lasting adaptive behavioral change occurs in response to (repeated) exposure to an olfactory cue. Relationships: is a type of associative learning [GO:0008306]; is a type of olfactory behavior [GO:0042048]